B-1 B cell lineage commitment [GO:0002336] (biological process) Definition: The process in which an immature B cell becomes committed to become a B-1 B cell. Sources: GOC:jal, ISBN:0781735149 Also known as: B-1 B lymphocyte lineage commitment, B-1 B-cell lineage commitment, B-1 B-lymphocyte lineage commitment Relationships: is a type of B cell lineage commitment [GO:0002326]; is part of GO:0001923